{
  "term_id": "GO:0005762",
  "term_label": "mitochondrial large ribosomal subunit",
  "gene_symbol": "MRPL27",
  "gene": "UniProtKB:Q9P0M9",
  "gene_name": "Large ribosomal subunit protein bL27m"
}